{
  "gene_name": "Endoplasmic reticulum transmembrane helix translocase",
  "gene": "UniProtKB:Q9HD20",
  "term_id": "GO:0005789",
  "term_label": "endoplasmic reticulum membrane",
  "gene_symbol": "ATP13A1"
}